{
  "term_id": "UNKNOWN:0003",
  "term_label": "Unknown cellular component",
  "gene_symbol": "SLX4IP",
  "gene": "UniProtKB:Q5VYV7",
  "gene_name": "Protein SLX4IP"
}